{
  "gene_symbol": "CCS",
  "gene": "UniProtKB:O14618",
  "term_id": "UNKNOWN:0003",
  "term_label": "Unknown cellular component",
  "gene_name": "Copper chaperone for superoxide dismutase"
}